{
  "gene": "UniProtKB:Q13515",
  "term_id": "GO:0045109",
  "term_label": "intermediate filament organization",
  "gene_symbol": "BFSP2",
  "gene_name": "Phakinin"
}